{
  "gene_name": "E3 ubiquitin-protein ligase PPP1R11",
  "gene_symbol": "PPP1R11",
  "gene": "UniProtKB:O60927",
  "term_label": "Unknown biological process",
  "term_id": "UNKNOWN:0002"
}